aromatic amino acid family catabolic process [GO:0009074] (biological process) Relationships: is a type of aromatic amino acid metabolic process [GO:0009072]; is a type of carboxylic acid catabolic process [GO:0046395] Also known as: aromatic amino acid family breakdown, aromatic amino acid family catabolism, aromatic amino acid family degradation Sources: GOC:go_curators Subtypes: aromatic amino acid family catabolic process to alcohol via Ehrlich pathway [GO:0000949], GO:0000952, L-histidine catabolic process [GO:0006548], L-phenylalanine catabolic process [GO:0006559], L-tryptophan catabolic process [GO:0006569], GO:0006572, anthranilate catabolic process [GO:0043421], GO:1900829 Definition: The chemical reactions and pathways resulting in the breakdown of aromatic amino acid family, amino acids with aromatic ring (phenylalanine, tyrosine, tryptophan).